pyridoxine metabolic process [GO:0008614] (biological process) Sources: GOC:curators Relationships: is a type of vitamin B6 metabolic process [GO:0042816] Also known as: pyridoxine metabolism Definition: The chemical reactions and pathways involving pyridoxine, 2-methyl-3-hydroxy-4,5-bis(hydroxymethyl)pyridine, one of the vitamin B6 compounds. Pyridoxal, pyridoxamine and pyridoxine are collectively known as vitamin B6, and are efficiently converted to the biologically active form of vitamin B6, pyridoxal phosphate. Subtypes: pyridoxine biosynthetic process [GO:0008615]